male germ-line stem cell population maintenance [GO:0036098] (biological process) Definition: The process by which an organism or tissue maintains a population of male germ-line stem cells. Relationships: is a type of germ-line stem cell population maintenance [GO:0030718] References: PMID:21752937 Sources: GOC:sart